{
  "gene_symbol": "TXNDC8",
  "gene": "UniProtKB:Q6A555",
  "term_id": "GO:0005794",
  "term_label": "Golgi apparatus",
  "gene_name": "Thioredoxin domain-containing protein 8"
}